5-aminopentanamidase activity [GO:0047588] (molecular function) Definition: Catalysis of the reaction: 5-aminopentanamide + H2O = 5-aminopentanoate + NH3. Sources: EC:3.5.1.30, MetaCyc:5-AMINOPENTANAMIDASE-RXN Also known as: 5-aminonorvaleramidase activity, 5-aminopentanamide amidohydrolase activity, 5-aminovaleramidase activity Relationships: is a type of hydrolase activity, acting on carbon-nitrogen (but not peptide) bonds, in linear amides [GO:0016811]